temperature homeostasis [GO:0001659] (biological process) Definition: A homeostatic process in which an organism modulates its internal body temperature. Subtypes: heat generation [GO:0031649], heat dissipation [GO:0031653], homoiothermy [GO:0042309], circadian temperature homeostasis [GO:0060086], cold-induced thermogenesis [GO:0106106] Also known as: thermoregulation Relationships: is a type of GO:0048871 Sources: GOC:jl